SRP-dependent cotranslational protein targeting to membrane, signal sequence processing [GO:0006618] (biological process) Relationships: is a type of signal peptide processing [GO:0006465]; is part of SRP-dependent cotranslational protein targeting to membrane [GO:0006614] Also known as: SRP-dependent cotranslational membrane targeting, signal sequence processing, SRP-dependent cotranslational protein-membrane targeting, signal sequence processing, signal sequence processing during SRP-dependent cotranslational protein targeting to membrane Definition: The removal of the signal peptide from a nascent protein during cotranslational membrane targeting. Sources: ISBN:0815316194